{
  "term_label": "Unknown cellular component",
  "gene_name": "Uncharacterized protein C4orf54",
  "gene_symbol": "C4orf54",
  "gene": "UniProtKB:D6RIA3",
  "term_id": "UNKNOWN:0003"
}